{
  "gene_symbol": "SYT13",
  "gene_name": "Synaptotagmin-13",
  "term_id": "GO:0061891",
  "gene": "UniProtKB:Q7L8C5",
  "term_label": "calcium ion sensor activity"
}